{
  "term_id": "GO:0005886",
  "gene": "UniProtKB:O14827",
  "gene_name": "Ras-specific guanine nucleotide-releasing factor 2",
  "term_label": "plasma membrane",
  "gene_symbol": "RASGRF2"
}